{
  "gene": "UniProtKB:Q6NUQ1",
  "term_label": "retrograde vesicle-mediated transport, Golgi to endoplasmic reticulum",
  "gene_symbol": "RINT1",
  "term_id": "GO:0006890",
  "gene_name": "RAD50-interacting protein 1"
}